inositol 1,3,4,5 tetrakisphosphate binding [GO:0043533] (molecular function) Also known as: IP4 binding, InsP4 binding Definition: Binding to inositol 1,3,4,5 tetrakisphosphate. Relationships: is a type of anion binding [GO:0043168]; is a type of alcohol binding [GO:0043178] Sources: GOC:go_curators